{
  "term_id": "GO:0005615",
  "gene": "UniProtKB:O95750",
  "term_label": "extracellular space",
  "gene_symbol": "FGF19",
  "gene_name": "Fibroblast growth factor 19"
}